alpha-pinene catabolic process [GO:0046249] (BP) Relationships: is a type of alpha-pinene metabolic process [GO:0018867]; is a type of pinene catabolic process [GO:0033074] References: PMID:10192895, PMID:14736461, PMID:29414896 Definition: The chemical reactions and pathways resulting in the breakdown of alpha-pinene, a monoterpene that may be a significant factor affecting bacterial activities in nature. Also known as: alpha-pinene breakdown, alpha-pinene catabolism, alpha-pinene degradation